{
  "term_id": "GO:0005978",
  "gene_name": "Glycogen [starch] synthase, liver",
  "gene": "UniProtKB:P54840",
  "gene_symbol": "GYS2",
  "term_label": "glycogen biosynthetic process"
}